response to Thyroglobulin triiodothyronine [GO:1904016] (biological process) Definition: Any process that results in a change in state or activity of a cell or an organism (in terms of movement, secretion, enzyme production, gene expression, etc.) as a result of a Thyroglobulin triiodothyronine stimulus. References: PMID:7531505 Sources: GOC:TermGenie, GO_REF:0000071 Relationships: is a type of response to chemical [GO:0042221] Subtypes: GO:1904017